tRNA seleno-modification [GO:0070329] (biological process) References: PMID:14594807 Sources: GOC:jsg Definition: The substitution of a selenium atom for a sulfur atom in a ribonucleotide in a tRNA molecule. Relationships: is a type of selenium compound metabolic process [GO:0001887]; is a type of tRNA modification [GO:0006400] Also known as: tRNA base modification to selenouridine